{
  "term_label": "Unknown molecular function",
  "term_id": "UNKNOWN:0001",
  "gene": "UniProtKB:Q17R60",
  "gene_symbol": "IMPG1",
  "gene_name": "Interphotoreceptor matrix proteoglycan 1"
}